regulation of Lewy body formation [GO:0140122] (biological process) Subtypes: negative regulation of Lewy body formation [GO:0140123], positive regulation of Lewy body formation [GO:0140124] Relationships: is a type of regulation of inclusion body assembly [GO:0090083]; regulates GO:0140121 Sources: GOC:sl Definition: Any process that modulates the frequency, rate or extent of Lewy body formation.